xanthosine nucleotidase activity [GO:0072585] (molecular function) References: PMID:21235647 Sources: GOC:kad, MetaCyc:RXN0-363 Also known as: xanthosine ribohydrolase activity Definition: Catalysis of the reaction: xanthosine + H2O = D-ribose + xanthine. Relationships: is a type of GO:0008477